{
  "gene_symbol": "KCNT2",
  "term_id": "GO:0015271",
  "gene": "UniProtKB:Q6UVM3",
  "term_label": "outward rectifier potassium channel activity",
  "gene_name": "Potassium channel subfamily T member 2"
}